{
  "gene_name": "Transcription factor SOX-14",
  "gene": "UniProtKB:O95416",
  "term_id": "GO:0030182",
  "gene_symbol": "SOX14",
  "term_label": "neuron differentiation"
}